T cell proliferation [GO:0042098] (biological process) Relationships: is a type of GO:0042110; is a type of lymphocyte proliferation [GO:0046651] Definition: The expansion of a T cell population by cell division. Follows T cell activation. Subtypes: T cell homeostatic proliferation [GO:0001777], T cell proliferation involved in immune response [GO:0002309], immature T cell proliferation [GO:0033079], gamma-delta T cell proliferation [GO:0046630], alpha-beta T cell proliferation [GO:0046633], GO:0050798, memory T cell proliferation [GO:0061485] Regulation: positively regulated by positive regulation of T cell proliferation [GO:0042102]; regulated by regulation of T cell proliferation [GO:0042129]; negatively regulated by negative regulation of T cell proliferation [GO:0042130] Sources: GOC:jl Also known as: T lymphocyte proliferation, T-cell proliferation, T-lymphocyte proliferation